{
  "gene_symbol": "P2RY6",
  "gene_name": "P2Y purinoceptor 6",
  "term_label": "G protein-coupled UTP receptor activity",
  "term_id": "GO:0045030",
  "gene": "UniProtKB:Q15077"
}